negative regulation of protein homooligomerization [GO:0032463] (biological process) Relationships: is a type of GO:0032460; is a type of regulation of protein homooligomerization [GO:0032462]; negatively regulates protein homooligomerization [GO:0051260] Also known as: down regulation of protein homooligomerization, down-regulation of protein homooligomerization, downregulation of protein homooligomerization, inhibition of protein homooligomerization Subtypes: GO:1901094 Definition: Any process that stops, prevents, or reduces the frequency, rate or extent of protein homooligomerization. Sources: GOC:mah